posterior lateral line nerve glial cell morphogenesis involved in differentiation [GO:0048942] (biological process) Definition: The process in which the structures of a glial cell in the posterior lateral line nerve are generated and organized. This process occurs while the initially relatively unspecialized cell is acquiring the specialized features of a glial cell in the posterior lateral line nerve. Relationships: is a type of GO:0048938; BFO_0000050 posterior lateral line nerve glial cell development [GO:0048941] Sources: GOC:dgh